{
  "gene_name": "Disintegrin and metalloproteinase domain-containing protein 29",
  "term_label": "proteolysis",
  "gene": "UniProtKB:Q9UKF5",
  "term_id": "GO:0006508",
  "gene_symbol": "ADAM29"
}